{
  "term_label": "ATP hydrolysis activity",
  "gene": "UniProtKB:P54277",
  "gene_name": "PMS1 protein homolog 1",
  "term_id": "GO:0016887",
  "gene_symbol": "PMS1"
}